{
  "gene": "UniProtKB:O94927",
  "term_id": "UNKNOWN:0001",
  "gene_name": "HAUS augmin-like complex subunit 5",
  "gene_symbol": "HAUS5",
  "term_label": "Unknown molecular function"
}